{
  "term_label": "nucleus",
  "gene_name": "SERTA domain-containing protein 2",
  "gene_symbol": "SERTAD2",
  "term_id": "GO:0005634",
  "gene": "UniProtKB:Q14140"
}